{
  "gene": "UniProtKB:Q9HBU9",
  "term_label": "cAMP binding",
  "gene_symbol": "POPDC2",
  "gene_name": "Popeye domain-containing protein 2",
  "term_id": "GO:0030552"
}